{
  "gene_name": "Dipeptidase 3",
  "term_id": "GO:0005886",
  "gene": "UniProtKB:Q9H4B8",
  "gene_symbol": "DPEP3",
  "term_label": "plasma membrane"
}